{
  "gene_symbol": "CACNB4",
  "term_label": "calcium ion transport",
  "gene_name": "Voltage-dependent L-type calcium channel subunit beta-4",
  "gene": "UniProtKB:O00305",
  "term_id": "GO:0006816"
}